development of primary male sexual characteristics [GO:0046546] (biological process) Definition: The process whose specific outcome is the progression of the primary male sexual characteristics over time, from their formation to the mature structures. The primary male sexual characteristics are the testes, and they develop in response to sex hormone secretion. Sources: GOC:ai Relationships: is a type of GO:0045137; is part of male sex differentiation [GO:0046661]